{
  "gene": "UniProtKB:Q9C037",
  "term_label": "innate immune response",
  "gene_symbol": "TRIM4",
  "term_id": "GO:0045087",
  "gene_name": "E3 ubiquitin-protein ligase TRIM4"
}